cellular response to undecane [GO:1902785] (biological process) Definition: Any process that results in a change in state or activity of a cell (in terms of movement, secretion, enzyme production, gene expression, etc.) as a result of an undecane stimulus. Relationships: is a type of cellular response to alkane [GO:1902779]; is a type of response to undecane [GO:1902784] References: PMID:23826995 Sources: GOC:TermGenie, GOC:mengo_curators, GO_REF:0000071